{
  "gene_symbol": "ALKBH1",
  "gene": "UniProtKB:Q13686",
  "term_id": "GO:0035515",
  "gene_name": "Nucleic acid dioxygenase ALKBH1",
  "term_label": "oxidative RNA demethylase activity"
}